spindle pole body localization [GO:0070631] (biological process) Also known as: spindle pole body localisation, maintenance of spindle pole body localization Relationships: is a type of cellular localization [GO:0051641]; is a type of GO:0061842 Definition: Any process in which a spindle pole body is transported to, or maintained in, a specific location. A spindle pole body is a type of microtubule organizing center found in fungal cells. Subtypes: mitotic spindle pole body localization [GO:1990608] Sources: GOC:mah